{
  "gene": "UniProtKB:Q5VXU1",
  "term_id": "UNKNOWN:0001",
  "gene_symbol": "NKAIN2",
  "term_label": "Unknown molecular function",
  "gene_name": "Sodium_potassium-transporting ATPase subunit beta-1-interacting protein 2"
}